glucarate dehydratase activity [GO:0008872] (molecular function) Sources: EC:4.2.1.40 Definition: Catalysis of the reaction: D-glucarate = 5-dehydro-4-deoxy-D-glucarate + H2O. Also known as: D-glucarate dehydratase activity, D-glucarate hydro-lyase (5-dehydro-4-deoxy-D-glucarate-forming), D-glucarate hydro-lyase activity Relationships: is a type of hydro-lyase activity [GO:0016836]